{
  "term_label": "cytokine-mediated signaling pathway",
  "gene": "UniProtKB:Q01344",
  "gene_symbol": "IL5RA",
  "term_id": "GO:0019221",
  "gene_name": "Interleukin-5 receptor subunit alpha"
}